{
  "gene": "UniProtKB:A0N4X5",
  "gene_symbol": "TRAJ34",
  "gene_name": "HCG2039756 (Fragment)",
  "term_id": "UNKNOWN:0002",
  "term_label": "Unknown biological process"
}